{
  "gene_name": "Metallothionein-1E",
  "term_id": "GO:0010273",
  "term_label": "detoxification of copper ion",
  "gene": "UniProtKB:P04732",
  "gene_symbol": "MT1E"
}